{
  "gene_name": "Chromatin assembly factor 1 subunit A",
  "term_label": "Unknown molecular function",
  "gene_symbol": "CHAF1A",
  "gene": "UniProtKB:Q13111",
  "term_id": "UNKNOWN:0001"
}